{
  "gene_symbol": "PTTG2",
  "term_label": "nucleus",
  "term_id": "GO:0005634",
  "gene_name": "Securin-2",
  "gene": "UniProtKB:Q9NZH5"
}